tropane alkaloid biosynthetic process [GO:0009710] (biological process) Sources: GOC:ai, ISBN:0198506732 Relationships: is a type of alkaloid biosynthetic process [GO:0009821] Definition: The chemical reactions and pathways resulting in the breakdown of tropane alkaloids, compounds containing the 8-methyl-8-azabicyclo(3.2.1)octane ring system. Also known as: tropane alkaloid anabolism, tropane alkaloid biosynthesis, tropane alkaloid formation, tropane alkaloid synthesis Subtypes: cocaine biosynthetic process [GO:0050799], scopolamine biosynthetic process [GO:1900991], atropine biosynthetic process [GO:1901051], GO:1901869, ecgonone methyl ester biosynthetic process [GO:1901872]